lipoprotein catabolic process [GO:0042159] (biological process) Subtypes: protein depalmitoylation [GO:0002084], protein depalmitoleylation [GO:1990697] Also known as: lipoprotein breakdown, lipoprotein catabolism, lipoprotein degradation Definition: The chemical reactions and pathways resulting in the breakdown of any conjugated, water-soluble protein in which the covalently attached nonprotein group consists of a lipid or lipids. Sources: ISBN:0198506732 Relationships: is a type of protein catabolic process [GO:0030163]; is a type of lipoprotein metabolic process [GO:0042157]